{
  "gene": "UniProtKB:Q15274",
  "term_label": "quinolinate catabolic process",
  "gene_name": "Nicotinate-nucleotide pyrophosphorylase [carboxylating]",
  "term_id": "GO:0034213",
  "gene_symbol": "QPRT"
}